{
  "gene": "UniProtKB:Q9NQV5",
  "term_id": "GO:0000978",
  "term_label": "RNA polymerase II cis-regulatory region sequence-specific DNA binding",
  "gene_symbol": "PRDM11",
  "gene_name": "PR domain-containing protein 11"
}